digestive tract morphogenesis [GO:0048546] (biological process) Subtypes: endodermal digestive tract morphogenesis [GO:0061031] References: PMID:12618131 Sources: GOC:dph, GOC:go_curators Definition: The process in which the anatomical structures of the digestive tract are generated and organized. The digestive tract is the anatomical structure through which food passes and is processed. Also known as: gut morphogenesis, alimentary canal morphogenesis, digestive tube morphogenesis, gastrointestinal tract morphogenesis, intestinal morphogenesis Relationships: is a type of tube morphogenesis [GO:0035239]; is part of digestive tract development [GO:0048565]